{
  "term_id": "GO:1903898",
  "gene_symbol": "NCK2",
  "term_label": "negative regulation of PERK-mediated unfolded protein response",
  "gene": "UniProtKB:O43639",
  "gene_name": "Cytoplasmic protein NCK2"
}